{
  "gene": "UniProtKB:A6NIE9",
  "gene_name": "Putative serine protease 29",
  "term_label": "extracellular space",
  "gene_symbol": "PRSS29P",
  "term_id": "GO:0005615"
}